{
  "gene_symbol": "A1CF",
  "gene_name": "APOBEC1 complementation factor",
  "term_label": "mRNA binding",
  "gene": "UniProtKB:Q9NQ94",
  "term_id": "GO:0003729"
}